{
  "gene_symbol": "FADS3",
  "term_id": "GO:0016020",
  "gene": "UniProtKB:Q9Y5Q0",
  "gene_name": "Fatty acid desaturase 3",
  "term_label": "membrane"
}